{
  "gene_name": "Gamma-aminobutyric acid receptor subunit alpha-3",
  "term_id": "GO:0022851",
  "term_label": "GABA-gated chloride ion channel activity",
  "gene": "UniProtKB:P34903",
  "gene_symbol": "GABRA3"
}